cerebellar granular layer formation [GO:0021684] (biological process) Definition: The process that gives rise to the cerebellar granule layer. This process pertains to the initial formation of a structure from unspecified parts. The granular layer is the innermost layer of the cerebellar cortex. This layer contains densely packed small neurons, mostly granule cells. Some Golgi cells are found at the outer border. Granule neurons send parallel fibers to the upper molecular layer, where they synapse with Purkinje cell dendrites. Mossy fibers from the pontine nuclei in the white matter synapse with granule cell axons, Golgi cell axons and unipolar brush interneuron axons at cerebellar glomeruli in the granule cell layer. Sources: GOC:cls, GOC:dgh, GOC:dph, GOC:jid, GO_REF:0000021 Relationships: is a type of anatomical structure formation involved in morphogenesis [GO:0048646]; is part of cerebellar granular layer morphogenesis [GO:0021683]; is part of cerebellar cortex formation [GO:0021697]